beta-catenin destruction complex assembly [GO:1904885] (biological process) Relationships: is a type of GO:0065003 Definition: The aggregation, arrangement and bonding together of a set of components to form a beta-catenin destruction complex. References: PMID:17143292, PMID:23169527 Sources: GOC:PARL, GOC:TermGenie, GOC:bf, GO_REF:0000079 Also known as: APC-Axin-1-beta-catenin complex assembly, APC-Axin-1-beta-catenin complex formation, Axin-APC-beta-catenin-GSK3B complex assembly, Axin-APC-beta-catenin-GSK3B complex formation, BDC assembly, BDC formation, beta-catenin degradation complex assembly, beta-catenin degradation complex formation, beta-catenin destruction complex formation, 23S APC complex assembly, 23S APC complex formation, destruction complex formation